{
  "term_id": "UNKNOWN:0003",
  "gene": "UniProtKB:Q8NGM9",
  "term_label": "Unknown cellular component",
  "gene_name": "Olfactory receptor 8D4",
  "gene_symbol": "OR8D4"
}